{
  "gene_name": "FERM domain-containing protein 4A",
  "term_label": "bicellular tight junction",
  "gene": "UniProtKB:Q9P2Q2",
  "term_id": "GO:0005923",
  "gene_symbol": "FRMD4A"
}